alphav-beta3 integrin-ADAM23 complex [GO:0071067] (CC) Also known as: ITGAV-ITGB3-ADAM23 complex References: PMID:10749942 Definition: A protein complex that consists of an alphav-beta3 integrin complex bound to the transmembrane metallopeptidase ADAM23. Relationships: is a type of GO:0098797; is a type of catalytic complex [GO:1902494]